alphaV-beta3 integrin-paxillin-Pyk2 complex [GO:0071097] (cellular component) Definition: A protein complex that consists of an alphaV-beta3 integrin complex bound to paxillin and the FAK-related kinase Pyk2. References: PMID:11683411 Also known as: ITGAV-ITGB3-PXN-PTK2b complex Relationships: is a type of GO:0098797